NADP+ biosynthetic process [GO:0006741] (BP) Also known as: NADP (oxidized) biosynthesis, NADP (oxidized) biosynthetic process, NADP (reduced) biosynthesis, NADP (reduced) biosynthetic process, NADP anabolism, NADP biosynthesis, NADP biosynthetic process, NADP formation, NADP synthesis, NADPH biosynthesis, NADPH biosynthetic process, nicotinamide adenine dinucleotide phosphate biosynthesis, nicotinamide adenine dinucleotide phosphate biosynthetic process, oxidized NADP biosynthesis, oxidized NADP biosynthetic process, oxidized nicotinamide adenine dinucleotide phosphate biosynthesis, oxidized nicotinamide adenine dinucleotide phosphate biosynthetic process, reduced NADP biosynthesis, reduced NADP biosynthetic process, reduced nicotinamide adenine dinucleotide phosphate biosynthesis, reduced nicotinamide adenine dinucleotide phosphate biosynthetic process Definition: The chemical reactions and pathways resulting in the formation of nicotinamide adenine dinucleotide phosphate (NADP+), a coenzyme that interconverts with its reduced form, NADPH, in many redox and biosynthetic reactions. Sources: GOC:mah Relationships: is a type of purine nucleotide biosynthetic process [GO:0006164]; is a type of GO:0006739; is a type of nicotinamide nucleotide biosynthetic process [GO:0019359]